beta-alanine transport [GO:0001762] (biological process) Sources: GOC:hjd Relationships: is a type of neutral amino acid transport [GO:0015804]; is a type of carboxylic acid transport [GO:0046942]; is a type of nitrogen compound transport [GO:0071705] Definition: The directed movement of beta-alanine, 3-aminopropanoic acid, into, out of or within a cell, or between cells, by means of some agent such as a transporter or pore.